{
  "term_label": "Unknown biological process",
  "gene_name": "Chronophin",
  "gene_symbol": "PDXP",
  "gene": "UniProtKB:Q96GD0",
  "term_id": "UNKNOWN:0002"
}